ER to Golgi ceramide transport [GO:0035621] (biological process) Relationships: is a type of intracellular lipid transport [GO:0032365]; is a type of ceramide transport [GO:0035627] Also known as: ER to Golgi ceramide translocation, endoplasmic reticulum to Golgi ceramide transport, non-vesicular ceramide trafficking References: PMID:14685229 Sources: GOC:sart Definition: The directed movement of a ceramide from the endoplasmic reticulum (ER) to the Golgi. Ceramides are a class of lipid composed of sphingosine linked to a fatty acid.